{
  "term_id": "GO:0030202",
  "gene_symbol": "NAGLU",
  "gene_name": "Alpha-N-acetylglucosaminidase",
  "term_label": "heparin proteoglycan metabolic process",
  "gene": "UniProtKB:P54802"
}